{
  "term_id": "GO:0006955",
  "gene_symbol": "PECAM1",
  "term_label": "immune response",
  "gene": "UniProtKB:P16284",
  "gene_name": "Platelet endothelial cell adhesion molecule"
}